negative regulation of amniotic stem cell differentiation [GO:2000798] (biological process) Relationships: is a type of negative regulation of mesenchymal stem cell differentiation [GO:2000740]; is a type of regulation of amniotic stem cell differentiation [GO:2000797]; negatively regulates amniotic stem cell differentiation [GO:0097086] Definition: Any process that stops, prevents or reduces the frequency, rate or extent of amniotic stem cell differentiation. Sources: GOC:obol